{
  "term_id": "UNKNOWN:0002",
  "gene": "UniProtKB:Q96EI5",
  "gene_symbol": "TCEAL4",
  "gene_name": "Transcription elongation factor A protein-like 4",
  "term_label": "Unknown biological process"
}